{
  "gene": "UniProtKB:Q9H799",
  "gene_name": "Ciliogenesis and planar polarity effector 1",
  "gene_symbol": "CPLANE1",
  "term_label": "Unknown molecular function",
  "term_id": "UNKNOWN:0001"
}